{
  "gene_symbol": "LDHAL6B",
  "term_label": "mitochondrion",
  "term_id": "GO:0005739",
  "gene_name": "L-lactate dehydrogenase A-like 6B",
  "gene": "UniProtKB:Q9BYZ2"
}